platelet dense tubular network membrane [GO:0031095] (cellular component) Definition: The lipid bilayer surrounding the platelet dense tubular network. References: PMID:1322202 Sources: GOC:mah Relationships: is a type of bounding membrane of organelle [GO:0098588]; is part of GO:0031094